{
  "gene": "UniProtKB:Q9Y383",
  "term_label": "U2-type prespliceosome",
  "gene_symbol": "LUC7L2",
  "gene_name": "Putative RNA-binding protein Luc7-like 2",
  "term_id": "GO:0071004"
}